{
  "gene_symbol": "METTL22",
  "term_id": "GO:0005634",
  "term_label": "nucleus",
  "gene": "UniProtKB:Q9BUU2",
  "gene_name": "Methyltransferase-like protein 22"
}